{
  "term_id": "UNKNOWN:0002",
  "gene_symbol": "ANXA7",
  "gene_name": "Annexin A7",
  "gene": "UniProtKB:P20073",
  "term_label": "Unknown biological process"
}